{
  "gene_symbol": "AZI2",
  "term_id": "UNKNOWN:0001",
  "gene_name": "5-azacytidine-induced protein 2",
  "term_label": "Unknown molecular function",
  "gene": "UniProtKB:Q9H6S1"
}